{
  "gene": "UniProtKB:Q9H3P2",
  "gene_symbol": "NELFA",
  "gene_name": "Negative elongation factor A",
  "term_id": "GO:0032021",
  "term_label": "NELF complex"
}